L-fuculokinase activity [GO:0008737] (molecular function) Sources: EC:2.7.1.51, RHEA:12376 Relationships: is a type of phosphotransferase activity, alcohol group as acceptor [GO:0016773]; is a type of carbohydrate kinase activity [GO:0019200] Definition: Catalysis of the reaction: L-fuculose + ATP = L-fuculose 1-phosphate + ADP + 2 H+. Also known as: ATP:L-fuculose 1-phosphotransferase activity, L-fuculokinase (phosphorylating), L-fuculose kinase activity